regulation of phagocytosis [GO:0050764] (biological process) Sources: GOC:ai Subtypes: negative regulation of phagocytosis [GO:0050765], GO:0050766, regulation of phagocytosis, engulfment [GO:0060099], regulation of apoptotic cell clearance [GO:2000425] Definition: Any process that modulates the frequency, rate or extent of phagocytosis, the process in which phagocytes engulf external particulate material. Relationships: is a type of GO:0030100; regulates GO:0006909